{
  "term_label": "nucleus",
  "gene": "UniProtKB:Q99966",
  "term_id": "GO:0005634",
  "gene_name": "Cbp_p300-interacting transactivator 1",
  "gene_symbol": "CITED1"
}